{
  "gene": "UniProtKB:Q9Y698",
  "term_label": "postsynaptic neurotransmitter receptor diffusion trapping",
  "gene_symbol": "CACNG2",
  "gene_name": "Voltage-dependent calcium channel gamma-2 subunit",
  "term_id": "GO:0098970"
}